{
  "gene_symbol": "RB1",
  "term_id": "GO:0030154",
  "gene_name": "Retinoblastoma-associated protein",
  "gene": "UniProtKB:P06400",
  "term_label": "cell differentiation"
}